{
  "term_id": "GO:0017116",
  "term_label": "single-stranded DNA helicase activity",
  "gene_symbol": "MCM5",
  "gene": "UniProtKB:P33992",
  "gene_name": "DNA replication licensing factor MCM5"
}